{
  "gene_symbol": "HPD",
  "term_id": "GO:0000139",
  "gene": "UniProtKB:P32754",
  "term_label": "Golgi membrane",
  "gene_name": "4-hydroxyphenylpyruvate dioxygenase"
}